{
  "term_id": "GO:0005680",
  "gene_name": "Cell division cycle protein 20 homolog",
  "gene_symbol": "CDC20",
  "term_label": "anaphase-promoting complex",
  "gene": "UniProtKB:Q12834"
}